{
  "term_id": "GO:0030054",
  "gene_symbol": "SPTBN4",
  "gene_name": "Spectrin beta chain, non-erythrocytic 4",
  "term_label": "cell junction",
  "gene": "UniProtKB:Q9H254"
}